{
  "term_id": "GO:0035196",
  "gene": "UniProtKB:Q9UGR2",
  "gene_name": "Zinc finger CCCH domain-containing protein 7B",
  "term_label": "miRNA processing",
  "gene_symbol": "ZC3H7B"
}